{
  "term_label": "vesicle-mediated transport",
  "gene": "UniProtKB:Q6DN90",
  "gene_symbol": "IQSEC1",
  "term_id": "GO:0016192",
  "gene_name": "IQ motif and SEC7 domain-containing protein 1"
}